{
  "term_id": "GO:0005829",
  "gene_symbol": "SSB",
  "term_label": "cytosol",
  "gene_name": "Lupus La protein",
  "gene": "UniProtKB:P05455"
}